{
  "gene_symbol": "MYCL",
  "term_label": "regulation of transcription by RNA polymerase II",
  "gene_name": "Protein L-Myc",
  "gene": "UniProtKB:P12524",
  "term_id": "GO:0006357"
}